{
  "gene_name": "Caspase recruitment domain-containing protein 10",
  "term_id": "GO:0007165",
  "term_label": "signal transduction",
  "gene_symbol": "CARD10",
  "gene": "UniProtKB:Q9BWT7"
}